{
  "term_id": "GO:0005856",
  "gene": "UniProtKB:Q6NY19",
  "term_label": "cytoskeleton",
  "gene_name": "KN motif and ankyrin repeat domain-containing protein 3",
  "gene_symbol": "KANK3"
}